{
  "term_id": "UNKNOWN:0002",
  "gene": "UniProtKB:Q9H6E4",
  "gene_name": "Coiled-coil domain-containing protein 134",
  "gene_symbol": "CCDC134",
  "term_label": "Unknown biological process"
}